{
  "gene_symbol": "WWP2",
  "gene": "UniProtKB:O00308",
  "term_id": "GO:0061629",
  "gene_name": "NEDD4-like E3 ubiquitin-protein ligase WWP2",
  "term_label": "RNA polymerase II-specific DNA-binding transcription factor binding"
}